{
  "term_label": "positive regulation of DNA-templated transcription",
  "gene_symbol": "ZNF318",
  "gene": "UniProtKB:Q5VUA4",
  "term_id": "GO:0045893",
  "gene_name": "Zinc finger protein 318"
}